mast cell activation [GO:0045576] (biological process) Regulation: regulated by GO:0033003; negatively regulated by GO:0033004; positively regulated by positive regulation of mast cell activation [GO:0033005] Relationships: is a type of myeloid leukocyte activation [GO:0002274] Definition: The change in morphology and behavior of a mast cell resulting from exposure to a cytokine, chemokine, soluble factor, or to (at least in mammals) an antigen which the mast cell has specifically bound via IgE bound to Fc-epsilonRI receptors. Subtypes: mast cell activation involved in immune response [GO:0002279] Sources: GOC:mgi_curators, ISBN:0781735149